embryo sac central cell differentiation [GO:0009559] (biological process) Definition: The process in which the two uncellularized polar nuclei cellularize, fuse and acquire the specialized features of a mononucleate diploid central cell. Also known as: embryo sac endosperm mother cell differentiation, female gametophyte central cell differentiation Regulation: regulated by regulation of embryo sac central cell differentiation [GO:0045691]; negatively regulated by negative regulation of embryo sac central cell differentiation [GO:0045692]; positively regulated by positive regulation of embryo sac central cell differentiation [GO:0045693] Sources: GOC:jid, GOC:mtg_plant Relationships: is a type of cell differentiation [GO:0030154]; BFO_0000050 megagametogenesis [GO:0009561]